{
  "term_id": "GO:0000977",
  "gene_name": "LIM_homeobox protein Lhx4",
  "term_label": "RNA polymerase II transcription regulatory region sequence-specific DNA binding",
  "gene_symbol": "LHX4",
  "gene": "UniProtKB:Q969G2"
}